{
  "term_id": "UNKNOWN:0002",
  "term_label": "Unknown biological process",
  "gene_name": "Attractin",
  "gene": "UniProtKB:O75882",
  "gene_symbol": "ATRN"
}